negative regulation of chondrocyte development [GO:0061182] (biological process) Sources: GOC:BHF, GOC:dph Subtypes: negative regulation of chondrocyte hypertrophy [GO:1903042] Definition: Any process that decreases the rate, frequency, or extent of the process whose specific outcome is the progression of a chondrocyte over time, from its commitment to its mature state. Chondrocyte development does not include the steps involved in committing a chondroblast to a chondrocyte fate. Relationships: is a type of GO:0010721; is a type of negative regulation of chondrocyte differentiation [GO:0032331]; is a type of regulation of chondrocyte development [GO:0061181]; negatively regulates chondrocyte development [GO:0002063]